{
  "gene": "UniProtKB:Q8TCN5",
  "term_id": "GO:0003700",
  "term_label": "DNA-binding transcription factor activity",
  "gene_name": "Zinc finger protein 507",
  "gene_symbol": "ZNF507"
}